{
  "term_label": "Unknown biological process",
  "gene_symbol": "COPS7B",
  "gene_name": "COP9 signalosome complex subunit 7b",
  "gene": "UniProtKB:Q9H9Q2",
  "term_id": "UNKNOWN:0002"
}